{
  "gene_symbol": "PON2",
  "gene_name": "Serum paraoxonase_arylesterase 2",
  "gene": "UniProtKB:Q15165",
  "term_id": "GO:0004064",
  "term_label": "arylesterase activity"
}